DNA replication factor A complex [GO:0005662] (cellular component) Definition: A conserved heterotrimeric complex that binds nonspecifically to single-stranded DNA and is required for multiple processes in eukaryotic DNA metabolism, including DNA replication, DNA repair, and recombination. In all eukaryotic organisms examined the complex is composed of subunits of approximately 70, 30, and 14 kDa. Also known as: RPA, replication protein A Relationships: is a type of nuclear protein-containing complex [GO:0140513]; is part of nuclear replisome [GO:0043601] References: PMID:9242902